{
  "term_label": "anatomical structure morphogenesis",
  "gene_name": "Forkhead box protein C1",
  "gene_symbol": "FOXC1",
  "term_id": "GO:0009653",
  "gene": "UniProtKB:Q12948"
}